vascular endothelial growth factor receptor signaling pathway [GO:0048010] (biological process) Subtypes: vascular endothelial growth factor receptor-1 signaling pathway [GO:0036323], vascular endothelial growth factor receptor-2 signaling pathway [GO:0036324], vascular endothelial growth factor receptor-3 signaling pathway [GO:0036325], positive regulation of endothelial cell chemotaxis by VEGF-activated vascular endothelial growth factor receptor signaling pathway [GO:0038033], vascular endothelial growth factor receptor signaling pathway involved in lymphatic endothelial cell fate commitment [GO:0060851] Relationships: is a type of cell surface receptor protein tyrosine kinase signaling pathway [GO:0007169] Also known as: VEGF receptor signaling pathway, VEGF receptor signalling pathway, VEGFR signaling pathway Regulation: regulated by regulation of vascular endothelial growth factor receptor signaling pathway [GO:0030947]; negatively regulated by negative regulation of vascular endothelial growth factor receptor signaling pathway [GO:0030948]; RO_0002213 by positive regulation of vascular endothelial growth factor receptor signaling pathway [GO:0030949] Sources: GOC:ceb, GOC:signaling Definition: The series of molecular signals initiated by a ligand binding to a vascular endothelial growth factor receptor (VEGFR) on the surface of the target cell, and ending with the regulation of a downstream cellular process, e.g. transcription. Note: In GO, a gene product with 'vascular endothelial growth factor-activated receptor activity ; GO:0005021' necessarily binds VEGF to transduce a signal. In contrast, the VEGFR refers to PR:000001971. To represent cross-talk between ligands and receptors, signaling pathways in GO are starting to be named after the receptor and/or the signal. GO:0048010 is for annotation of any pathway in which a ligand (VEGF or an alternative growth factor) binds and activates a VEGFR (PR:000001971). For annotation of signaling pathways where a VEGF binds to a cell surface receptor (VEGFR, PDGFR etc.), consider 'vascular endothelial growth factor signaling pathway ; GO:0038084'.